{
  "term_id": "GO:0019706",
  "gene_symbol": "ZDHHC9",
  "term_label": "protein-cysteine S-palmitoyltransferase activity",
  "gene_name": "Palmitoyltransferase ZDHHC9",
  "gene": "UniProtKB:Q9Y397"
}